{
  "term_id": "GO:0071805",
  "term_label": "potassium ion transmembrane transport",
  "gene": "UniProtKB:Q9NZV8",
  "gene_name": "Potassium voltage-gated channel subfamily D member 2",
  "gene_symbol": "KCND2"
}